{
  "gene": "UniProtKB:Q5VSY0",
  "gene_symbol": "GKAP1",
  "term_id": "UNKNOWN:0003",
  "gene_name": "G kinase-anchoring protein 1",
  "term_label": "Unknown cellular component"
}